thymidylate synthase activity [GO:0004799] (molecular function) Definition: Catalysis of the reaction: 5,10-methylenetetrahydrofolate + dUMP = 7,8-dihydrofolate + thymidylate. Relationships: is a type of 5,10-methylenetetrahydrofolate-dependent methyltransferase activity [GO:0042083] Sources: EC:2.1.1.45, RHEA:12104 Also known as: 5,10-methylenetetrahydrofolate:dUMP C-methyltransferase activity, TMP synthetase activity, dTMP synthase activity, methylenetetrahydrofolate:dUMP C-methyltransferase activity, thymidylate synthetase activity